{
  "term_id": "UNKNOWN:0003",
  "term_label": "Unknown cellular component",
  "gene_symbol": "A6NHS1",
  "gene_name": "Putative uncharacterized protein ENSP00000347057",
  "gene": "UniProtKB:A6NHS1"
}